{
  "gene": "UniProtKB:Q8TCD5",
  "gene_name": "5'(3')-deoxyribonucleotidase, cytosolic type",
  "term_id": "UNKNOWN:0003",
  "gene_symbol": "NT5C",
  "term_label": "Unknown cellular component"
}